{
  "gene": "UniProtKB:Q96EY7",
  "gene_symbol": "PTCD3",
  "gene_name": "Small ribosomal subunit protein mS39",
  "term_id": "GO:0005739",
  "term_label": "mitochondrion"
}